{
  "gene_name": "E3 ubiquitin-protein ligase parkin",
  "gene_symbol": "PRKN",
  "gene": "UniProtKB:O60260",
  "term_label": "Golgi apparatus",
  "term_id": "GO:0005794"
}